{
  "gene": "UniProtKB:Q58FF8",
  "term_id": "GO:0051082",
  "term_label": "unfolded protein binding",
  "gene_name": "Putative heat shock protein HSP 90-beta 2",
  "gene_symbol": "HSP90AB2P"
}